{
  "term_id": "GO:0004758",
  "gene_symbol": "SPTSSA",
  "term_label": "serine C-palmitoyltransferase activity",
  "gene": "UniProtKB:Q969W0",
  "gene_name": "Serine palmitoyltransferase small subunit A"
}